{
  "gene_symbol": "POLD4",
  "term_id": "GO:0043625",
  "term_label": "delta DNA polymerase complex",
  "gene": "UniProtKB:Q9HCU8",
  "gene_name": "DNA polymerase delta subunit 4"
}